halogenated hydrocarbon catabolic process [GO:0042206] (biological process) Sources: GOC:ai, GOC:krc Definition: The chemical reactions and pathways resulting in the breakdown of halogenated hydrocarbons, compounds derived from hydrocarbons by replacing one or more hydrogen atoms with halogen atoms. Relationships: is a type of GO:0042178; is a type of halogenated hydrocarbon metabolic process [GO:0042197] Subtypes: 1,2-dichloroethane catabolic process [GO:0019260], carbon tetrachloride catabolic process [GO:0019382], chlorinated hydrocarbon catabolic process [GO:0042205] Also known as: halogenated hydrocarbon breakdown, halogenated hydrocarbon catabolism, halogenated hydrocarbon degradation